{
  "gene_symbol": "XIRP1",
  "gene": "UniProtKB:Q702N8",
  "term_label": "actin filament binding",
  "term_id": "GO:0051015",
  "gene_name": "Xin actin-binding repeat-containing protein 1"
}